late viral transcription [GO:0019086] (biological process) Definition: The transcription of the final group of viral genes of the viral life cycle, following middle transcription, or where middle transcription doesn't occur, following early transcription. Involves the transcription of genes encoding structural proteins. Also known as: late viral mRNA transcription Relationships: is a type of viral transcription [GO:0019083] Sources: GOC:bf, GOC:jh2, GOC:jl